{
  "gene_symbol": "PPFIA3",
  "gene_name": "Liprin-alpha-3",
  "gene": "UniProtKB:O75145",
  "term_label": "synapse organization",
  "term_id": "GO:0050808"
}